{
  "term_label": "Unknown molecular function",
  "term_id": "UNKNOWN:0001",
  "gene": "UniProtKB:Q6P9G4",
  "gene_name": "Transmembrane protein 154",
  "gene_symbol": "TMEM154"
}